{
  "gene_symbol": "KIF15",
  "term_id": "GO:0008017",
  "gene_name": "Kinesin-like protein KIF15",
  "gene": "UniProtKB:Q9NS87",
  "term_label": "microtubule binding"
}